karyosome formation [GO:0061988] (biological process) Relationships: is a type of GO:0061982; is a type of chromosome organization involved in meiotic cell cycle [GO:0070192]; is part of gamete generation [GO:0007276] References: PMID:19696886 Definition: The chromosome organization process in which meiotic chromosomes in the germ cell nucleus cluster together to form a compact spherical structure called the karyosome. Subtypes: oocyte karyosome formation [GO:0030717], sperm karyosome formation [GO:0061989]